regulation of type I hypersensitivity [GO:0001810] (biological process) Sources: ISBN:0781735149 Relationships: is a type of regulation of hypersensitivity [GO:0002883]; is a type of regulation of immunoglobulin mediated immune response [GO:0002889]; RO_0002211 type I hypersensitivity [GO:0016068] Subtypes: negative regulation of type I hypersensitivity [GO:0001811], GO:0001812 Definition: Any process that modulates the frequency, rate, or extent of type I hypersensitivity, a type of inflammatory response.